symbiont-mediated degradation of host mRNA [GO:0039595] (biological process) Relationships: is a type of symbiont-mediated perturbation of host gene expression [GO:0039656] References: PMID:12163576, PMID:16477041, PMID:17360652, PMID:22696660 Also known as: induction by virus of catabolism of host mRNA, induction by virus of host mRNA catabolic process, induction of host mRNA decay, promotion of host mRNA degradation, viral induction of host mRNA decay, virus-mediated mRNA decay Definition: The process in which a virus increases the frequency, rate or extent of the breakdown of host messenger RNA (mRNA).